{
  "gene": "UniProtKB:Q9Y371",
  "term_id": "GO:0061024",
  "gene_name": "Endophilin-B1",
  "gene_symbol": "SH3GLB1",
  "term_label": "membrane organization"
}